{
  "gene_symbol": "CDH5",
  "gene": "UniProtKB:P33151",
  "term_id": "GO:0044331",
  "gene_name": "Cadherin-5",
  "term_label": "cell-cell adhesion mediated by cadherin"
}